regulation of natural killer cell mediated cytotoxicity [GO:0042269] (biological process) Definition: Any process that modulates the frequency, rate, or extent of natural killer cell mediated cytotoxicity. Sources: GOC:add, ISBN:0781735149 Relationships: is a type of regulation of leukocyte mediated cytotoxicity [GO:0001910]; is a type of GO:0002715; RO_0002211 natural killer cell mediated cytotoxicity [GO:0042267] Also known as: regulation of NK cell mediated cell death, regulation of NK cell mediated cell killing, regulation of natural killer cell mediated cell death, regulation of natural killer cell mediated cell killing, regulation of NK cell mediated cytolysis, regulation of NK cell mediated cytotoxicity, regulation of natural killer cell mediated cytolysis, regulation of natural killer-cell mediated cytolysis Subtypes: regulation of natural killer cell mediated cytotoxicity directed against tumor cell target [GO:0002858], regulation of natural killer cell degranulation [GO:0043321], negative regulation of natural killer cell mediated cytotoxicity [GO:0045953], positive regulation of natural killer cell mediated cytotoxicity [GO:0045954]